{
  "term_label": "regulation of transcription by RNA polymerase II",
  "gene": "UniProtKB:Q99990",
  "term_id": "GO:0006357",
  "gene_name": "Transcription cofactor vestigial-like protein 1",
  "gene_symbol": "VGLL1"
}